response to acadesine [GO:1904101] (biological process) References: PMID:20802119 Sources: GOC:TermGenie, GOC:mr, GO_REF:0000071 Relationships: is a type of GO:1901698; is a type of response to oxygen-containing compound [GO:1901700] Definition: Any process that results in a change in state or activity of a cell or an organism (in terms of movement, secretion, enzyme production, gene expression, etc.) as a result of an acadesine stimulus. Subtypes: cellular response to acadesine [GO:1904102]